L-ornithine transmembrane transporter activity [GO:0000064] (molecular function) Also known as: L-ornithine transporter activity, histidine/arginine/lysine/ornithine porter activity Relationships: is_a L-amino acid transmembrane transporter activity [GO:0015179]; is part of L-ornithine transmembrane transport [GO:1903352] Definition: Enables the transfer of L-ornithine from one side of a membrane to the other. L-ornithine is 2,5-diaminopentanoic acid. Subtypes: putrescine:ornithine antiporter activity [GO:0015496], GO:0097627 Sources: GOC:ai, GOC:mtg_transport, ISBN:0815340729